{
  "term_id": "GO:0070382",
  "gene": "UniProtKB:Q8N9I0",
  "term_label": "exocytic vesicle",
  "gene_symbol": "SYT2",
  "gene_name": "Synaptotagmin-2"
}